valencene synthase activity [GO:0102905] (MF) Sources: EC:4.2.3.73, GOC:pz Relationships: is a type of GO:0016838 Definition: Catalysis of the reaction: 2-trans,6-trans-farnesyl diphosphate(3-) = (+)-valencene + diphosphoric acid.